anaerobic cobalamin biosynthetic process [GO:0019251] (biological process) Sources: GOC:go_curators Also known as: anaerobic cobalamin anabolism, anaerobic cobalamin biosynthesis, anaerobic cobalamin formation, anaerobic cobalamin synthesis, anaerobic vitamin B12 biosynthesis, anaerobic vitamin B12 biosynthetic process, cobalamin biosynthesis, anaerobic, cobalamin biosynthetic process, anaerobic, vitamin B12 biosynthesis, anaerobic, vitamin B12 biosynthetic process, anaerobic Relationships: is a type of cobalamin biosynthetic process [GO:0009236] Definition: The chemical reactions and pathways resulting in the formation of cobalamin (vitamin B12) in the absence of oxygen.